{
  "gene_name": "T-cell leukemia homeobox protein 1",
  "term_label": "DNA-binding transcription factor activity, RNA polymerase II-specific",
  "gene_symbol": "TLX1",
  "term_id": "GO:0000981",
  "gene": "UniProtKB:P31314"
}